{
  "gene": "UniProtKB:Q8WX77",
  "gene_name": "Insulin-like growth factor-binding protein-like 1",
  "term_label": "regulation of signal transduction",
  "gene_symbol": "IGFBPL1",
  "term_id": "GO:0009966"
}